longitudinal sarcoplasmic reticulum lumen [GO:0014803] (cellular component) Sources: GOC:mtg_muscle Relationships: is a type of sarcoplasmic reticulum lumen [GO:0033018]; is part of longitudinal sarcoplasmic reticulum [GO:0014801] Definition: The region between the inner and outer lipid bilayers of the longitudinal sarcoplasmic reticulum envelope. The longitudinal sarcoplasmic reticulum lumen is continuous with the lumen contained within the terminal cisternae.